{
  "term_id": "UNKNOWN:0002",
  "term_label": "Unknown biological process",
  "gene": "UniProtKB:Q8IZD9",
  "gene_name": "Dedicator of cytokinesis protein 3",
  "gene_symbol": "DOCK3"
}